{
  "gene_name": "60S ribosome subunit biogenesis protein NIP7 homolog",
  "term_label": "Unknown molecular function",
  "term_id": "UNKNOWN:0001",
  "gene": "UniProtKB:Q9Y221",
  "gene_symbol": "NIP7"
}